positive regulation of protein maturation [GO:1903319] (biological process) Subtypes: GO:0010954, positive regulation of N-terminal peptidyl-methionine acetylation [GO:1904665], positive regulation of protein activation cascade [GO:2000259], positive regulation of N-terminal peptidyl-lysine acetylation [GO:2000761] Also known as: up regulation of protein maturation, up-regulation of protein maturation, upregulation of protein maturation, activation of protein maturation Definition: Any process that activates or increases the frequency, rate or extent of protein maturation. Relationships: is a type of GO:0010628; is a type of positive regulation of protein metabolic process [GO:0051247]; is a type of regulation of protein maturation [GO:1903317]; positively regulates protein maturation [GO:0051604] Sources: GOC:TermGenie, GOC:vw, GO_REF:0000058